{
  "gene": "UniProtKB:Q3KNV8",
  "gene_name": "Polycomb group RING finger protein 3",
  "term_id": "UNKNOWN:0001",
  "gene_symbol": "PCGF3",
  "term_label": "Unknown molecular function"
}